{
  "term_id": "UNKNOWN:0003",
  "gene_symbol": "KL",
  "gene": "UniProtKB:Q9UEF7",
  "term_label": "Unknown cellular component",
  "gene_name": "Klotho"
}